{
  "gene": "UniProtKB:O43741",
  "term_label": "nucleus",
  "gene_name": "5'-AMP-activated protein kinase subunit beta-2",
  "term_id": "GO:0005634",
  "gene_symbol": "PRKAB2"
}